positive regulation of methane biosynthetic process from methanethiol [GO:1900347] (biological process) Also known as: up regulation of methane biosynthetic process from methanethiol, up-regulation of methane biosynthetic process from methanethiol, upregulation of methane biosynthetic process from methanethiol, activation of methane biosynthetic process from methanethiol Sources: GOC:TermGenie, GOC:mengo_curators Definition: Any process that activates or increases the frequency, rate or extent of methane biosynthetic process from methanethiol. Relationships: is a type of regulation of methane biosynthetic process from methanethiol [GO:1900345]; is a type of positive regulation of alkane biosynthetic process [GO:1901579]; is a type of positive regulation of cellular respiration [GO:1901857]; positively regulates methane biosynthetic process from methanethiol [GO:2001133]